{
  "term_label": "antigen binding",
  "gene_symbol": "IGHV3-35",
  "gene_name": "Probable non-functional immunoglobulin heavy variable 3-35",
  "term_id": "GO:0003823",
  "gene": "UniProtKB:A0A0C4DH35"
}